{
  "gene_name": "Transmembrane domain-containing protein TMIGD3",
  "gene_symbol": "TMIGD3",
  "gene": "UniProtKB:P0DMS9",
  "term_id": "GO:0005886",
  "term_label": "plasma membrane"
}